{
  "term_id": "UNKNOWN:0001",
  "term_label": "Unknown molecular function",
  "gene": "UniProtKB:Q86T23",
  "gene_symbol": "CROCCP2",
  "gene_name": "Putative ciliary rootlet coiled-coil protein-like 1 protein"
}